{
  "gene": "UniProtKB:Q14019",
  "gene_symbol": "COTL1",
  "term_id": "GO:0005884",
  "term_label": "actin filament",
  "gene_name": "Coactosin-like protein"
}